{
  "term_label": "cell morphogenesis",
  "gene": "UniProtKB:Q6ZTQ4",
  "term_id": "GO:0000902",
  "gene_name": "Cadherin-related family member 3",
  "gene_symbol": "CDHR3"
}